positive regulation of dendritic cell dendrite assembly [GO:2000549] (biological process) Definition: Any process that activates or increases the frequency, rate or extent of dendritic cell dendrite assembly. Relationships: is a type of positive regulation of plasma membrane bounded cell projection assembly [GO:0120034]; is a type of GO:2000547; positively regulates dendritic cell dendrite assembly [GO:0097026] Sources: GOC:obol Also known as: positive regulation of dendritic extension